3-chloro THPH synthase activity [GO:0106266] (molecular function) References: PMID:20231486 Sources: RHEA:64356 Definition: Catalysis of the reaction: 2,4,6-trihydroxyphenylhexan-1-one + chloride + FADH2 + O2 = (3-chloro-2,4,6-trihydroxyphenyl)hexan-1-one + FAD + H+ + 2 H2O. Relationships: is a type of oxidoreductase activity, acting on paired donors, with incorporation or reduction of molecular oxygen, reduced flavin or flavoprotein as one donor, and incorporation of one atom of oxygen [GO:0016712]